{
  "gene_name": "Myomegalin",
  "gene_symbol": "PDE4DIP",
  "term_id": "GO:1903358",
  "gene": "UniProtKB:Q5VU43",
  "term_label": "regulation of Golgi organization"
}